{
  "gene_name": "Hemoglobin subunit zeta",
  "gene": "UniProtKB:P02008",
  "term_label": "hemoglobin complex",
  "gene_symbol": "HBZ",
  "term_id": "GO:0005833"
}